{
  "gene_symbol": "CSRP3",
  "term_label": "Z disc",
  "term_id": "GO:0030018",
  "gene": "UniProtKB:P50461",
  "gene_name": "Cysteine and glycine-rich protein 3"
}